{
  "term_label": "Unknown molecular function",
  "term_id": "UNKNOWN:0001",
  "gene_symbol": "FAM184B",
  "gene_name": "Protein FAM184B",
  "gene": "UniProtKB:Q9ULE4"
}